{
  "term_label": "insulin receptor signaling pathway",
  "gene": "UniProtKB:O15530",
  "gene_name": "3-phosphoinositide-dependent protein kinase 1",
  "term_id": "GO:0008286",
  "gene_symbol": "PDPK1"
}